{
  "gene_name": "Mediator of RNA polymerase II transcription subunit 17",
  "term_id": "GO:0003712",
  "gene": "UniProtKB:Q9NVC6",
  "term_label": "transcription coregulator activity",
  "gene_symbol": "MED17"
}